{
  "gene": "UniProtKB:Q9H213",
  "gene_name": "Melanoma-associated antigen H1",
  "term_id": "UNKNOWN:0001",
  "gene_symbol": "MAGEH1",
  "term_label": "Unknown molecular function"
}